{
  "gene_symbol": "TEK",
  "term_label": "cell surface receptor protein tyrosine kinase signaling pathway",
  "gene": "UniProtKB:Q02763",
  "term_id": "GO:0007169",
  "gene_name": "Angiopoietin-1 receptor"
}